vitamin metabolic process [GO:0006766] (biological process) Definition: The chemical reactions and pathways involving vitamins. Vitamin is a general term for a number of unrelated organic substances that occur in many foods in small amounts and that are necessary in trace amounts for the normal metabolic functioning of the body. Vitamins may be water-soluble or fat-soluble and usually serve as components of coenzyme systems. Sources: GOC:ai Also known as: vitamin metabolism Relationships: is a type of small molecule metabolic process [GO:0044281] Subtypes: vitamin biosynthetic process [GO:0009110], vitamin catabolic process [GO:0009111] Regulation: regulated by GO:0030656; positively regulated by positive regulation of vitamin metabolic process [GO:0046136]; negatively regulated by negative regulation of vitamin metabolic process [GO:0046137]